{
  "gene_symbol": "CASP2",
  "term_label": "cysteine-type endopeptidase activity",
  "gene_name": "Caspase-2",
  "term_id": "GO:0004197",
  "gene": "UniProtKB:P42575"
}